{
  "gene_symbol": "NRBF2",
  "gene": "UniProtKB:Q96F24",
  "term_id": "UNKNOWN:0001",
  "term_label": "Unknown molecular function",
  "gene_name": "Nuclear receptor-binding factor 2"
}